{
  "term_label": "Unknown molecular function",
  "gene_symbol": "LRRIQ3",
  "gene": "UniProtKB:A6PVS8",
  "term_id": "UNKNOWN:0001",
  "gene_name": "Leucine-rich repeat and IQ domain-containing protein 3"
}